{
  "term_id": "GO:0035435",
  "gene_symbol": "SLC25A10",
  "term_label": "phosphate ion transmembrane transport",
  "gene": "UniProtKB:Q9UBX3",
  "gene_name": "Mitochondrial dicarboxylate carrier"
}